regulation of blood coagulation, common pathway [GO:2000260] (BP) Definition: Any process that modulates the frequency, rate or extent of blood coagulation, common pathway. Sources: GOC:mah Relationships: is a type of GO:0030193; is a type of GO:2000257; regulates blood coagulation, common pathway [GO:0072377] Subtypes: negative regulation of blood coagulation, common pathway [GO:2000261], positive regulation of blood coagulation, common pathway [GO:2000262]